{
  "term_id": "UNKNOWN:0003",
  "term_label": "Unknown cellular component",
  "gene": "UniProtKB:Q9UHL3",
  "gene_symbol": "FAM153A",
  "gene_name": "Protein FAM153A"
}